1-phosphatidyl-1D-myo-inositol 4,5-bisphosphate metabolic process [GO:1902633] (biological process) Subtypes: GO:1902634, GO:1902635 Definition: The chemical reactions and pathways involving 1-phosphatidyl-1D-myo-inositol 4,5-bisphosphate. Also known as: 1-phosphatidyl-1D-myo-inositol 4,5-bisphosphate metabolism Note: Phosphatidylinositol-4,5-bisphosphate, PtdIns(4,5)P(2) common name. Relationships: is a type of GO:0046488 References: PMID:22562153 Sources: GOC:TermGenie, GOC:di, GO_REF:0000068